{
  "gene_symbol": "CCPG1",
  "term_id": "UNKNOWN:0001",
  "gene": "UniProtKB:Q9ULG6",
  "gene_name": "Cell cycle progression protein 1",
  "term_label": "Unknown molecular function"
}